{
  "term_id": "GO:0051764",
  "gene_name": "Brain-specific angiogenesis inhibitor 1-associated protein 2",
  "gene_symbol": "BAIAP2",
  "term_label": "actin crosslink formation",
  "gene": "UniProtKB:Q9UQB8"
}